{
  "term_label": "cadherin binding",
  "gene_name": "Cadherin-23",
  "gene_symbol": "CDH23",
  "gene": "UniProtKB:Q9H251",
  "term_id": "GO:0045296"
}